{
  "term_label": "histone H3K4 methyltransferase activity",
  "term_id": "GO:0042800",
  "gene": "UniProtKB:Q9NQV7",
  "gene_symbol": "PRDM9",
  "gene_name": "Histone-lysine N-methyltransferase PRDM9"
}